{
  "term_id": "GO:0000981",
  "term_label": "DNA-binding transcription factor activity, RNA polymerase II-specific",
  "gene": "UniProtKB:Q9Y2V3",
  "gene_symbol": "RAX",
  "gene_name": "Retinal homeobox protein Rx"
}